{
  "term_id": "GO:0015816",
  "gene": "UniProtKB:Q495N2",
  "gene_name": "Proton-coupled amino acid transporter 3",
  "gene_symbol": "SLC36A3",
  "term_label": "glycine transport"
}